{
  "gene_symbol": "ERBB2",
  "term_label": "epidermal growth factor receptor signaling pathway",
  "term_id": "GO:0007173",
  "gene": "UniProtKB:P04626",
  "gene_name": "Receptor tyrosine-protein kinase erbB-2"
}